{
  "term_label": "positive regulation of cholesterol efflux",
  "gene_name": "Oxysterols receptor LXR-alpha",
  "gene_symbol": "NR1H3",
  "term_id": "GO:0010875",
  "gene": "UniProtKB:Q13133"
}